nuclear exosome (RNase complex) [GO:0000176] (cellular component) Also known as: eukaryotic exosome multienzyme ribonuclease complex, nuclear exosome (ribonuclease complex), nuclear exosome multienzyme ribonuclease complex Definition: A ribonuclease complex that has 3-prime to 5-prime processive and distributive hydrolytic exoribonuclease activity and endoribonuclease activity, producing 5-prime-phosphomonoesters. Participates in a multitude of cellular RNA processing and degradation events preventing nuclear export and/or translation of aberrant RNAs. Restricted to processing linear and circular single-stranded RNAs (ssRNA) only. RNAs with complex secondary structures may have to be unwound or pre-processed by co-factors prior to entering the complex, esp if the 3-prime end is structured. Subtypes: nucleolar exosome (RNase complex) [GO:0101019] Relationships: is a type of GO:0000178; is a type of nuclear protein-containing complex [GO:0140513]; is part of GO:0031981 References: PMID:17174896, PMID:20531386, PMID:26726035